{
  "gene": "UniProtKB:Q8WY50",
  "gene_name": "Placenta-specific protein 4",
  "term_id": "UNKNOWN:0001",
  "gene_symbol": "PLAC4",
  "term_label": "Unknown molecular function"
}